{
  "gene_name": "Actin-related protein 3",
  "gene": "UniProtKB:P61158",
  "term_label": "actin filament binding",
  "gene_symbol": "ACTR3",
  "term_id": "GO:0051015"
}